positive regulation of monocyte extravasation [GO:2000439] (BP) Relationships: is a type of positive regulation of cellular extravasation [GO:0002693]; is a type of GO:0071677; is a type of regulation of monocyte extravasation [GO:2000437]; positively regulates monocyte extravasation [GO:0035696] Sources: GOC:obol Definition: Any process that activates or increases the frequency, rate or extent of monocyte extravasation.